{
  "term_label": "TORC1 signaling",
  "gene": "UniProtKB:Q15418",
  "gene_name": "Ribosomal protein S6 kinase alpha-1",
  "term_id": "GO:0038202",
  "gene_symbol": "RPS6KA1"
}